positive regulation of complement-dependent cytotoxicity [GO:1903661] (biological process) Relationships: is a type of positive regulation of cell killing [GO:0031343]; is a type of regulation of complement-dependent cytotoxicity [GO:1903659]; positively regulates complement-dependent cytotoxicity [GO:0097278] Also known as: up regulation of complement-dependent cytotoxicity, up-regulation of complement-dependent cytotoxicity, upregulation of complement-dependent cytotoxicity, activation of complement-dependent cytotoxicity References: PMID:24280217 Sources: GOC:TermGenie, GO_REF:0000058 Definition: Any process that activates or increases the frequency, rate or extent of complement-dependent cytotoxicity.